negative regulation of UDP-N-acetylglucosamine biosynthetic process [GO:0106279] (biological process) Definition: Any process that stops, prevents or reduces the frequency, rate or extent of the UDP-N-acetylglucosamine biosynthetic process. References: PMID:32579556 Also known as: negative regulation of UDP-GlcNAc biosynthesis, negative regulation of UDP-GlcNAc biosynthetic process, negative regulation of UDP-N-acetylglucosamine anabolism, negative regulation of UDP-N-acetylglucosamine biosynthesis, negative regulation of UDP-N-acetylglucosamine formation, negative regulation of UDP-N-acetylglucosamine synthesis Relationships: is_a negative regulation of biosynthetic process [GO:0009890]; is a type of negative regulation of nucleobase-containing compound metabolic process [GO:0045934]; is a type of negative regulation of phosphate metabolic process [GO:0045936]; is a type of GO:0062014; is_a GO:0106278; negatively regulates UDP-N-acetylglucosamine biosynthetic process [GO:0006048]